{
  "term_label": "cytoplasm",
  "gene_symbol": "PPP1R9B",
  "term_id": "GO:0005737",
  "gene": "UniProtKB:Q96SB3",
  "gene_name": "Neurabin-2"
}